opioid peptide activity [GO:0001515] (molecular function) Relationships: is_a receptor ligand activity [GO:0048018] Sources: ISBN:0198506732 Definition: Naturally occurring peptide that is an opioid (any non-alkaloid having an opiate-like effect that can be reversed by naloxone or other recognized morphine antagonist). These include Leu- and Met-enkephalin, dynorphin and neoendorphin, alpha, beta, gamma and delta endorphins formed from beta-lipotropin, various pronase-resistant peptides such as beta casamorphin, and other peptides whose opiate-like action seems to be indirect.